insulin catabolic process [GO:1901143] (biological process) Relationships: is a type of protein catabolic process [GO:0030163]; is a type of insulin metabolic process [GO:1901142] Sources: GOC:TermGenie Definition: The chemical reactions and pathways resulting in the breakdown of insulin. Also known as: insulin breakdown, insulin catabolism, insulin degradation